{
  "term_label": "group III metabotropic glutamate receptor activity",
  "gene": "UniProtKB:Q14831",
  "gene_symbol": "GRM7",
  "term_id": "GO:0001642",
  "gene_name": "Metabotropic glutamate receptor 7"
}